{
  "gene_name": "Tyrosine-protein kinase JAK2",
  "gene_symbol": "JAK2",
  "gene": "UniProtKB:O60674",
  "term_id": "GO:0060397",
  "term_label": "growth hormone receptor signaling pathway via JAK-STAT"
}